{
  "term_id": "GO:1990247",
  "gene_name": "YTH domain-containing family protein 2",
  "gene_symbol": "YTHDF2",
  "gene": "UniProtKB:Q9Y5A9",
  "term_label": "N6-methyladenosine-containing RNA reader activity"
}